{
  "gene_name": "Gephyrin",
  "term_id": "GO:0006777",
  "gene_symbol": "GPHN",
  "gene": "UniProtKB:Q9NQX3",
  "term_label": "Mo-molybdopterin cofactor biosynthetic process"
}